female pigmentation [GO:0048095] (biological process) Definition: Establishment of a pattern of pigment in females. Regulation: regulated by regulation of female pigmentation [GO:0048089]; negatively regulated by negative regulation of female pigmentation [GO:0048090]; positively regulated by positive regulation of female pigmentation [GO:0048091] Sources: GOC:jid Relationships: is_a GO:0048071; is part of GO:0046660